{
  "term_id": "GO:0006887",
  "gene_name": "Syntaxin-2",
  "gene": "UniProtKB:P32856",
  "gene_symbol": "STX2",
  "term_label": "exocytosis"
}